collagen-activated signaling pathway [GO:0038065] (biological process) Subtypes: GO:0038063 Relationships: is a type of GO:0007166 References: PMID:21568710 Sources: GOC:bf, GOC:uh Also known as: collagen-activated signalling pathway Definition: The series of molecular signals initiated by collagen binding to a cell surface receptor, and ending with the regulation of a downstream cellular process, e.g. transcription.